metanephric glomerular parietal epithelial cell development [GO:0072246] (biological process) Definition: The process whose specific outcome is the progression of a metanephric glomerular parietal epithelial cell over time, from its formation to the mature structure. Metanephric glomerular parietal epithelial cells are specialized epithelial cells that form tight junctions as a barrier to protein transport. Sources: GOC:mtg_kidney_jan10 Also known as: metanephric Bowman's capsule development Relationships: is a type of glomerular parietal epithelial cell development [GO:0072016]; is a type of metanephric glomerular epithelial cell development [GO:0072313]; is part of metanephric glomerular parietal epithelial cell differentiation [GO:0072245]